cholesterol 7-alpha-monooxygenase activity [GO:0008123] (molecular function) Relationships: is a type of steroid 7-alpha-hydroxylase activity [GO:0008387]; is a type of oxidoreductase activity, acting on paired donors, with incorporation or reduction of molecular oxygen, reduced flavin or flavoprotein as one donor, and incorporation of one atom of oxygen [GO:0016712] Sources: RHEA:21812 Also known as: cholesterol 7-alpha-hydroxylase activity, cytochrome P450 CYP7A1, cholesterol 7alpha-hydroxylase activity, cholesterol 7alpha-monooxygenase activity, cholesterol,NADPH:oxygen oxidoreductase (7alpha-hydroxylating) Definition: Catalysis of the reaction: cholesterol + O2 + reduced [NADPH--hemoprotein reductase] = 7alpha-hydroxycholesterol + H+ + H2O + oxidized [NADPH--hemoprotein reductase].